{
  "gene": "UniProtKB:Q30KP8",
  "gene_name": "Defensin beta 136",
  "term_label": "Unknown cellular component",
  "term_id": "UNKNOWN:0003",
  "gene_symbol": "DEFB136"
}